{
  "term_label": "protein N-linked glycosylation",
  "gene_name": "Keratinocyte-associated protein 2",
  "gene_symbol": "KRTCAP2",
  "gene": "UniProtKB:Q8N6L1",
  "term_id": "GO:0006487"
}